{
  "gene_name": "Proenkephalin-B",
  "term_id": "GO:0007600",
  "gene": "UniProtKB:P01213",
  "gene_symbol": "PDYN",
  "term_label": "sensory perception"
}